{
  "term_label": "Unknown biological process",
  "gene": "UniProtKB:A6NK89",
  "gene_name": "Ras association domain-containing protein 10",
  "term_id": "UNKNOWN:0002",
  "gene_symbol": "RASSF10"
}